{
  "gene_symbol": "GRIP2",
  "gene_name": "Glutamate receptor-interacting protein 2",
  "gene": "UniProtKB:Q9C0E4",
  "term_label": "neurotransmitter receptor transport, endosome to postsynaptic membrane",
  "term_id": "GO:0098887"
}